{
  "gene": "UniProtKB:Q3KR16",
  "term_id": "UNKNOWN:0002",
  "term_label": "Unknown biological process",
  "gene_symbol": "PLEKHG6",
  "gene_name": "Pleckstrin homology domain-containing family G member 6"
}